{
  "gene": "UniProtKB:Q13670",
  "gene_symbol": "PMS2P11",
  "term_label": "Unknown molecular function",
  "term_id": "UNKNOWN:0001",
  "gene_name": "Putative postmeiotic segregation increased 2-like protein 11"
}